{
  "gene_name": "T-cell surface glycoprotein CD1c",
  "gene_symbol": "CD1C",
  "term_id": "GO:0071723",
  "term_label": "lipopeptide binding",
  "gene": "UniProtKB:P29017"
}